regulation of interleukin-6 production [GO:0032675] (biological process) Relationships: is_a regulation of cytokine production [GO:0001817]; regulates interleukin-6 production [GO:0032635] Sources: GOC:mah Definition: Any process that modulates the frequency, rate, or extent of interleukin-6 production. Also known as: regulation of IL-6 production, regulation of interleukin-6 biosynthetic process Subtypes: negative regulation of interleukin-6 production [GO:0032715], GO:0032755